{
  "gene_name": "WD repeat-containing protein 17",
  "term_id": "UNKNOWN:0003",
  "gene": "UniProtKB:Q8IZU2",
  "gene_symbol": "WDR17",
  "term_label": "Unknown cellular component"
}